{
  "gene": "UniProtKB:Q9H2D1",
  "term_label": "FAD transmembrane transporter activity",
  "term_id": "GO:0015230",
  "gene_symbol": "SLC25A32",
  "gene_name": "Mitochondrial folate transporter_carrier"
}